phosphoglycerate mutase activity [GO:0004619] (molecular function) Sources: RHEA:15901 Also known as: PGM, 2,3-bisphosphoglycerate-dependent phosphoglycerate mutase activity, 2,3-bisphosphoglycerate-independent phosphoglycerate mutase activity, D-phosphoglycerate 2,3-phosphomutase activity, PGA mutase activity, PGAM activity, phosphoglycerate phosphomutase activity, phosphoglyceromutase activity Relationships: is a type of GO:0016868 Definition: Catalysis of the reaction: (2R)-2-phosphoglycerate = (2R)-3-phosphoglycerate.